{
  "gene_name": "Actin-related protein 6",
  "gene": "UniProtKB:Q9GZN1",
  "term_label": "nucleosome binding",
  "term_id": "GO:0031491",
  "gene_symbol": "ACTR6"
}